{
  "gene": "UniProtKB:Q9H169",
  "term_label": "neuron projection development",
  "gene_symbol": "STMN4",
  "term_id": "GO:0031175",
  "gene_name": "Stathmin-4"
}